chromatin insulator sequence binding [GO:0043035] (MF) Definition: Binding to a chromatin insulator sequence, a DNA sequence that prevents enhancer-mediated activation or repression of transcription. References: PMID:12783795 Sources: GOC:jl Relationships: is a type of chromatin DNA binding [GO:0031490]